{
  "term_id": "UNKNOWN:0001",
  "term_label": "Unknown molecular function",
  "gene_name": "CKLF-like MARVEL transmembrane domain-containing protein 2",
  "gene": "UniProtKB:Q8TAZ6",
  "gene_symbol": "CMTM2"
}